regulation of reductive pentose-phosphate cycle [GO:0080152] (biological process) Relationships: is a type of regulation of photosynthesis, dark reaction [GO:0010110]; regulates reductive pentose-phosphate cycle [GO:0019253] Subtypes: GO:0080153 References: PMID:17031544 Also known as: regulation of C3 photosynthesis, regulation of Calvin cycle Definition: Any process that modulates the frequency, rate or extent of reductive pentose-phosphate cycle.